{
  "gene_symbol": "NRSN2",
  "term_id": "GO:0030133",
  "gene_name": "Neurensin-2",
  "term_label": "transport vesicle",
  "gene": "UniProtKB:Q9GZP1"
}